{
  "term_id": "GO:0005509",
  "gene": "UniProtKB:Q14257",
  "gene_name": "Reticulocalbin-2",
  "term_label": "calcium ion binding",
  "gene_symbol": "RCN2"
}